alpha-humulene synthase activity [GO:0080017] (MF) Definition: Catalysis of the reaction: 2-trans,6-trans-farnesyl diphosphate = alpha-humulene + diphosphate. References: PMID:12566586, PMID:9442047 Sources: RHEA:31895 Relationships: is a type of cyclase activity [GO:0009975]; is_a sesquiterpene synthase activity [GO:0010334]